{
  "gene_name": "Secretoglobin family 1D member 1",
  "gene_symbol": "SCGB1D1",
  "term_id": "UNKNOWN:0002",
  "term_label": "Unknown biological process",
  "gene": "UniProtKB:O95968"
}